{
  "gene_symbol": "ITGB7",
  "term_label": "integrin complex",
  "gene": "UniProtKB:P26010",
  "gene_name": "Integrin beta-7",
  "term_id": "GO:0008305"
}